{
  "gene": "UniProtKB:Q9Y561",
  "gene_name": "Low-density lipoprotein receptor-related protein 12",
  "gene_symbol": "LRP12",
  "term_label": "Unknown molecular function",
  "term_id": "UNKNOWN:0001"
}